{
  "gene_symbol": "NUP155",
  "gene": "UniProtKB:O75694",
  "gene_name": "Nuclear pore complex protein Nup155",
  "term_label": "protein localization to nuclear inner membrane",
  "term_id": "GO:0036228"
}